{
  "gene_name": "Protein Jade-3",
  "term_label": "histone reader activity",
  "gene": "UniProtKB:Q92613",
  "gene_symbol": "JADE3",
  "term_id": "GO:0140566"
}